{
  "gene_symbol": "SDHA",
  "gene_name": "Succinate dehydrogenase [ubiquinone] flavoprotein subunit, mitochondrial",
  "term_label": "electron transfer activity",
  "term_id": "GO:0009055",
  "gene": "UniProtKB:P31040"
}